13-lipoxin reductase activity [GO:0036185] (molecular function) Definition: Catalysis of the reaction: 15-oxo-(5S,6R)-dihydroxy-(7E,9E,11Z,13E)-eicosatetraenoate + NADH + H+ = 15-oxo-(5S,6R)-dihydroxy-(7E,9E,11Z)-eicosatrienoate + NAD+. References: PMID:10837478 Sources: RHEA:41592 Relationships: is a type of GO:0016616